{
  "gene": "UniProtKB:O75146",
  "gene_name": "Huntingtin-interacting protein 1-related protein",
  "term_label": "regulation of apoptotic process",
  "gene_symbol": "HIP1R",
  "term_id": "GO:0042981"
}